{
  "term_label": "plasma membrane",
  "gene": "UniProtKB:Q8NGK0",
  "term_id": "GO:0005886",
  "gene_name": "Olfactory receptor 51G2",
  "gene_symbol": "OR51G2"
}